{
  "gene_symbol": "KCTD19",
  "gene": "UniProtKB:Q17RG1",
  "term_id": "UNKNOWN:0001",
  "gene_name": "BTB_POZ domain-containing protein KCTD19",
  "term_label": "Unknown molecular function"
}